{
  "term_label": "histone H4K16 deacetylase activity, NAD-dependent",
  "term_id": "GO:0046970",
  "gene_name": "NAD-dependent protein deacetylase sirtuin-1",
  "gene": "UniProtKB:Q96EB6",
  "gene_symbol": "SIRT1"
}